{
  "gene": "UniProtKB:Q53F39",
  "gene_symbol": "MPPE1",
  "term_id": "UNKNOWN:0002",
  "term_label": "Unknown biological process",
  "gene_name": "Metallophosphoesterase 1"
}